{
  "gene_symbol": "DLG3",
  "term_label": "chemical synaptic transmission",
  "gene_name": "Disks large homolog 3",
  "gene": "UniProtKB:Q92796",
  "term_id": "GO:0007268"
}